{
  "gene_name": "Nucleosome-remodeling factor subunit BPTF",
  "term_label": "NURF complex",
  "gene": "UniProtKB:Q12830",
  "gene_symbol": "BPTF",
  "term_id": "GO:0016589"
}